{
  "gene_name": "Solute carrier organic anion transporter family member 3A1",
  "term_label": "sodium-independent organic anion transport",
  "gene_symbol": "SLCO3A1",
  "gene": "UniProtKB:Q9UIG8",
  "term_id": "GO:0043252"
}